telencephalon development [GO:0021537] (biological process) Also known as: cerebrum development References: PMID:12626695 Sources: GOC:cls, GOC:dgh, GOC:dph, GOC:jid, GO_REF:0000021 Relationships: is a type of anatomical structure development [GO:0048856]; is part of forebrain development [GO:0030900] Definition: The process whose specific outcome is the progression of the telencephalon over time, from its formation to the mature structure. The telencephalon is the paired anteriolateral division of the prosencephalon plus the lamina terminalis from which the olfactory lobes, cerebral cortex, and subcortical nuclei are derived.